{
  "term_id": "GO:0090263",
  "gene": "UniProtKB:Q86T65",
  "gene_symbol": "DAAM2",
  "gene_name": "Disheveled-associated activator of morphogenesis 2",
  "term_label": "positive regulation of canonical Wnt signaling pathway"
}